{
  "term_id": "GO:0008298",
  "gene_name": "Double-stranded RNA-binding protein Staufen homolog 2",
  "term_label": "intracellular mRNA localization",
  "gene_symbol": "STAU2",
  "gene": "UniProtKB:Q9NUL3"
}